{
  "gene": "UniProtKB:Q9H1C3",
  "term_id": "UNKNOWN:0002",
  "gene_name": "Glycosyltransferase 8 domain-containing protein 2",
  "term_label": "Unknown biological process",
  "gene_symbol": "GLT8D2"
}